{
  "gene": "UniProtKB:Q9UHA4",
  "gene_symbol": "LAMTOR3",
  "term_id": "GO:0060090",
  "gene_name": "Ragulator complex protein LAMTOR3",
  "term_label": "molecular adaptor activity"
}